{
  "gene_symbol": "LIM2",
  "term_id": "UNKNOWN:0002",
  "gene": "UniProtKB:P55344",
  "term_label": "Unknown biological process",
  "gene_name": "Lens fiber membrane intrinsic protein"
}